formation of plant organ boundary [GO:0090691] (biological process) Definition: The regionalization process that specifies plant organ primordium boundaries resulting in a restriction of organogenesis to a limited spatial domain and keeping the organ separate from surrounding tissues. Subtypes: organ boundary specification between lateral organs and the meristem [GO:0010199], cotyledon boundary formation [GO:0090451], shoot organ boundary specification [GO:0090470] Sources: GOC:tb Relationships: is_a formation of anatomical boundary [GO:0048859]